{
  "gene": "UniProtKB:P26572",
  "term_label": "Golgi apparatus",
  "term_id": "GO:0005794",
  "gene_name": "Alpha-1,3-mannosyl-glycoprotein 2-beta-N-acetylglucosaminyltransferase",
  "gene_symbol": "MGAT1"
}